{
  "gene": "UniProtKB:Q7Z7G2",
  "gene_symbol": "CPLX4",
  "gene_name": "Complexin-4",
  "term_id": "GO:0050804",
  "term_label": "modulation of chemical synaptic transmission"
}